{
  "term_id": "UNKNOWN:0002",
  "gene_symbol": "IGLJ4",
  "term_label": "Unknown biological process",
  "gene_name": "Immunoglobulin lambda joining 4 (non-functional) (Fragment)",
  "gene": "UniProtKB:A0A0A0MTA1"
}